regulation of activation-induced cell death of T cells [GO:0070235] (biological process) Subtypes: GO:0070236, GO:0070237 Sources: GOC:add, ISBN:0781765196 Relationships: is a type of regulation of immune system process [GO:0002682]; is a type of regulation of T cell apoptotic process [GO:0070232]; regulates activation-induced cell death of T cells [GO:0006924] Also known as: regulation of AICD, regulation of activated T cell apoptosis, regulation of antigen-driven apoptosis, regulation of activation-induced cell death of T lymphocytes, regulation of activation-induced cell death of T-cells, regulation of activation-induced cell death of T-lymphocytes Definition: Any process that modulates the occurrence or rate of activation-induced cell death of T cells.